regulation of intrinsic apoptotic signaling pathway by p53 class mediator [GO:1902253] (biological process) References: PMID:15705871 Sources: GOC:BHF, GOC:TermGenie, GOC:mtg_apoptosis, GOC:rl Definition: Any process that modulates the frequency, rate or extent of intrinsic apoptotic signaling pathway by p53 class mediator. Also known as: regulation of intrinsic apoptotic signaling pathway by signal transduction by p53 class mediator, regulation of signal transduction by p53 class mediator resulting in induction of apoptosis Relationships: is a type of regulation of signal transduction by p53 class mediator [GO:1901796]; is_a regulation of intrinsic apoptotic signaling pathway [GO:2001242]; regulates intrinsic apoptotic signaling pathway by p53 class mediator [GO:0072332] Subtypes: regulation of intrinsic apoptotic signaling pathway in response to DNA damage by p53 class mediator [GO:1902165], GO:1902238, negative regulation of intrinsic apoptotic signaling pathway by p53 class mediator [GO:1902254], positive regulation of intrinsic apoptotic signaling pathway by p53 class mediator [GO:1902255]